{
  "gene": "UniProtKB:Q9C0B9",
  "gene_name": "Zinc finger CCHC domain-containing protein 2",
  "term_label": "Unknown cellular component",
  "term_id": "UNKNOWN:0003",
  "gene_symbol": "ZCCHC2"
}